DNA helicase activity [GO:0003678] (molecular function) Subtypes: four-way junction helicase activity [GO:0009378], GO:0017116, GO:0036121, GO:0043138, GO:0043139, GO:0061749 Relationships: is a type of GO:0004386; is a type of ATP-dependent activity, acting on DNA [GO:0008094] Sources: GOC:jl Also known as: ATP-dependent DNA helicase activity Definition: Unwinding of a DNA helix, driven by ATP hydrolysis.